{
  "term_id": "GO:0060337",
  "term_label": "type I interferon-mediated signaling pathway",
  "gene_symbol": "IFNAR2",
  "gene": "UniProtKB:P48551",
  "gene_name": "Interferon alpha_beta receptor 2"
}